negative regulation of male pigmentation [GO:0048092] (biological process) Definition: Any process that stops, prevents, or reduces the frequency, rate or extent of establishment of a pattern of pigment in males. Sources: GOC:jid Also known as: down regulation of male pigmentation, down-regulation of male pigmentation, downregulation of male pigmentation, inhibition of male pigmentation Relationships: is_a GO:0048086; is a type of regulation of male pigmentation [GO:0048088]; is a type of negative regulation of developmental process [GO:0051093]; is a type of negative regulation of multicellular organismal process [GO:0051241]; is a type of negative regulation of reproductive process [GO:2000242]; RO_0002212 GO:0048094